{
  "term_id": "GO:0030424",
  "gene_symbol": "SYT4",
  "gene_name": "Synaptotagmin-4",
  "term_label": "axon",
  "gene": "UniProtKB:Q9H2B2"
}